{
  "term_label": "lipid transporter activity",
  "term_id": "GO:0005319",
  "gene": "UniProtKB:O94911",
  "gene_symbol": "ABCA8",
  "gene_name": "ABC-type organic anion transporter ABCA8"
}